{
  "term_id": "GO:0071011",
  "gene_name": "Pre-mRNA-splicing factor 38B",
  "gene_symbol": "PRPF38B",
  "term_label": "precatalytic spliceosome",
  "gene": "UniProtKB:Q5VTL8"
}